cell fate determination [GO:0001709] (biological process) Relationships: is a type of cellular developmental process [GO:0048869]; BFO_0000050 cell fate commitment [GO:0045165] Regulation: regulated by GO:1905933; negatively regulated by negative regulation of cell fate determination [GO:1905934]; positively regulated by positive regulation of cell fate determination [GO:1905935] Sources: ISBN:0878932437 Subtypes: ectodermal cell fate determination [GO:0001713], pole cell fate determination [GO:0007278], neuroblast fate determination [GO:0007400], GO:0007402, GO:0007403, epithelial cell fate determination, open tracheal system [GO:0007425], endodermal cell fate determination [GO:0007493], mesodermal cell fate determination [GO:0007500], GO:0007518, muscle cell fate determination [GO:0007521], oocyte fate determination [GO:0030716], leading edge cell fate determination [GO:0035028], eosinophil fate determination [GO:0035858], compound eye cone cell fate determination [GO:0042680], GO:0046845, neuron fate determination [GO:0048664], stem cell fate determination [GO:0048867], cell fate determination involved in pattern specification [GO:0060582], endothelial cell fate determination [GO:0060848], cardiac cell fate determination [GO:0060913], vulval cell fate determination [GO:0072326] Definition: The cellular developmental process involved in cell fate commitment that occurs after cell fate specification, in which a cell is irreversibly committed to a cellular developmental fate which is heritable on cell division.